{
  "gene_name": "Armadillo-like helical domain-containing protein 3",
  "term_label": "Unknown molecular function",
  "term_id": "UNKNOWN:0001",
  "gene_symbol": "ARMH3",
  "gene": "UniProtKB:Q5T2E6"
}